phagosome acidification involved in apoptotic cell clearance [GO:0090390] (biological process) Relationships: is a type of phagosome acidification [GO:0090383]; is part of GO:0090386 Definition: Any process that reduces the pH of the phagosome, measured by the concentration of the hydrogen ion, and occurs as a part of apoptotic cell clearance. Sources: GOC:kmv, GOC:tb